regulation of peptide hormone secretion [GO:0090276] (biological process) Definition: Any process that modulates the rate, frequency, or extent of the regulated release of a peptide hormone from secretory granules. Sources: GOC:tb Relationships: is_a regulation of peptide secretion [GO:0002791]; is a type of regulation of hormone secretion [GO:0046883]; regulates GO:0030072 Subtypes: GO:0043397, regulation of insulin secretion [GO:0050796], regulation of corticotropin secretion [GO:0051459], GO:0060123, regulation of glucagon secretion [GO:0070092], GO:0090273, positive regulation of peptide hormone secretion [GO:0090277], GO:0090278, GO:1904362, GO:1904458, GO:2000612